regulation of kinin cascade [GO:0002256] (biological process) Sources: GOC:jal Relationships: is a type of GO:0002673; is a type of GO:2000257; regulates kinin cascade [GO:0002254] Definition: Any process that modulates the frequency, rate, or extent of the kinin cascade. Subtypes: negative regulation of kinin cascade [GO:0002257], positive regulation of kinin cascade [GO:0002258], regulation of tissue kallikrein-kinin cascade [GO:0002382], GO:0002529